isopentenol biosynthetic process [GO:1902934] (biological process) Also known as: isopentenol anabolism, isopentenol biosynthesis, isopentenol formation, isopentenol synthesis Definition: The chemical reactions and pathways resulting in the formation of isopentenol. Relationships: is_a olefinic compound biosynthetic process [GO:0120255] References: PMID:17693564 Sources: GOC:TermGenie, GOC:mengo_curators, GO_REF:0000068